response to superoxide [GO:0000303] (biological process) Relationships: is a type of response to oxygen radical [GO:0000305] Definition: Any process that results in a change in state or activity of a cell or an organism (in terms of movement, secretion, enzyme production, gene expression, etc.) as a result of a superoxide stimulus. Superoxide is the anion, oxygen-, formed by addition of one electron to dioxygen (O2) or any compound containing the superoxide anion. Sources: GOC:krc, ISBN:0198506732 Subtypes: cellular response to superoxide [GO:0071451]